{
  "term_id": "GO:0004143",
  "gene_name": "Diacylglycerol kinase epsilon",
  "gene": "UniProtKB:P52429",
  "term_label": "ATP-dependent diacylglycerol kinase activity",
  "gene_symbol": "DGKE"
}